{
  "term_id": "GO:0050729",
  "gene": "UniProtKB:Q9Y4H4",
  "term_label": "positive regulation of inflammatory response",
  "gene_symbol": "GPSM3",
  "gene_name": "G-protein-signaling modulator 3"
}